glomerulus vasculature development [GO:0072012] (biological process) Definition: The biological process whose specific outcome is the progression of a glomerulus vasculature from an initial condition to its mature state. This process begins with the formation of the glomerulus vasculature and ends with the mature structure. The glomerulus vasculature is composed of the tubule structures that carry blood or lymph in the glomerulus. Relationships: is_a blood vessel development [GO:0001568]; is a type of kidney vasculature development [GO:0061440]; BFO_0000050 glomerulus development [GO:0032835] Also known as: glomerulus capillary development Sources: GOC:mtg_kidney_jan10 Subtypes: GO:0061231, metanephric glomerulus vasculature development [GO:0072239]